germline ring canal formation [GO:0030725] (biological process) Also known as: ring canal formation Subtypes: female germline ring canal formation [GO:0007301], male germline ring canal formation [GO:0030726] Sources: ISBN:0879694238 Definition: Assembly of the cytoplasmic bridges between developing spermatogonial or oogonial cysts. Relationships: is a type of cellular process involved in reproduction in multicellular organism [GO:0022412]; is a type of intercellular bridge organization [GO:0043063]